{
  "gene_name": "Protein transport protein Sec16B",
  "term_label": "ER to Golgi transport vesicle membrane",
  "gene": "UniProtKB:Q96JE7",
  "gene_symbol": "SEC16B",
  "term_id": "GO:0012507"
}